{
  "term_id": "GO:0060090",
  "gene_name": "Proteasome adapter and scaffold protein ECM29",
  "term_label": "molecular adaptor activity",
  "gene": "UniProtKB:Q5VYK3",
  "gene_symbol": "ECPAS"
}